{
  "term_label": "chemoattractant activity",
  "term_id": "GO:0042056",
  "gene_symbol": "VEGFA",
  "gene": "UniProtKB:P15692",
  "gene_name": "Vascular endothelial growth factor A, long form"
}